{
  "term_id": "UNKNOWN:0001",
  "term_label": "Unknown molecular function",
  "gene": "UniProtKB:Q9H0C5",
  "gene_symbol": "BTBD1",
  "gene_name": "BTB_POZ domain-containing protein 1"
}